{
  "gene_name": "Integrin alpha-E",
  "gene_symbol": "ITGAE",
  "term_label": "integrin-mediated signaling pathway",
  "term_id": "GO:0007229",
  "gene": "UniProtKB:P38570"
}